{
  "term_id": "GO:0006457",
  "gene_name": "Nuclear migration protein nudC",
  "gene_symbol": "NUDC",
  "gene": "UniProtKB:Q9Y266",
  "term_label": "protein folding"
}